{
  "gene": "UniProtKB:P04000",
  "gene_name": "Long-wave-sensitive opsin 1",
  "gene_symbol": "OPN1LW",
  "term_label": "G protein-coupled receptor signaling pathway",
  "term_id": "GO:0007186"
}